melatonin receptor activity [GO:0008502] (molecular function) Relationships: is a type of G protein-coupled receptor activity [GO:0004930] Sources: GOC:ai, ISBN:0198506732 Definition: Combining with melatonin, N-acetyl-5-methoxytryptamine, to initiate a change in cell activity. Melatonin is a neuroendocrine substance that stimulates the aggregation of melanosomes in melanophores, thus lightening the skin.